response to alkyl hydroperoxide [GO:0033195] (biological process) Sources: GOC:mah Relationships: is a type of response to hydroperoxide [GO:0033194] Subtypes: cellular response to alkyl hydroperoxide [GO:0071448], GO:0072735 Definition: Any process that results in a change in state or activity of a cell or an organism (in terms of movement, secretion, enzyme production, gene expression, etc.) as a result of an alkyl hydroperoxide stimulus. Alkyl hydroperoxides are monosubstitution products of hydrogen peroxide, HOOH, where the substituent is an alkyl group.